{
  "gene_symbol": "PAX2",
  "term_id": "GO:0006357",
  "term_label": "regulation of transcription by RNA polymerase II",
  "gene_name": "Paired box protein Pax-2",
  "gene": "UniProtKB:Q02962"
}